{
  "gene": "UniProtKB:O00712",
  "term_id": "GO:0005634",
  "gene_name": "Nuclear factor 1 B-type",
  "gene_symbol": "NFIB",
  "term_label": "nucleus"
}